{
  "gene_name": "Unconventional prefoldin RPB5 interactor 1",
  "gene_symbol": "URI1",
  "gene": "UniProtKB:O94763",
  "term_id": "GO:0042771",
  "term_label": "intrinsic apoptotic signaling pathway in response to DNA damage by p53 class mediator"
}